{
  "term_id": "GO:0031638",
  "gene_symbol": "F9",
  "gene": "UniProtKB:P00740",
  "gene_name": "Coagulation factor IX",
  "term_label": "zymogen activation"
}